kringle domain binding [GO:0036143] (molecular function) Sources: GOC:yaf, Wikipedia:Kringle_domain Definition: Binding to a kringle domain. Kringle domains are protein domains that fold into large loops stabilized by 3 disulfide linkages, and are important in protein-protein interactions with blood coagulation factors. Relationships: is a type of protein domain specific binding [GO:0019904]